{
  "gene_name": "Angiopoietin-like protein 8",
  "gene_symbol": "ANGPTL8",
  "term_label": "triglyceride homeostasis",
  "gene": "UniProtKB:Q6UXH0",
  "term_id": "GO:0070328"
}